{
  "term_label": "regulation of neutrophil migration",
  "gene_name": "Ras-related C3 botulinum toxin substrate 1",
  "gene": "UniProtKB:P63000",
  "term_id": "GO:1902622",
  "gene_symbol": "RAC1"
}